{
  "gene": "UniProtKB:Q9H693",
  "term_id": "UNKNOWN:0002",
  "gene_name": "Uncharacterized protein C16orf95",
  "gene_symbol": "C16orf95",
  "term_label": "Unknown biological process"
}